{
  "gene": "UniProtKB:P59537",
  "term_label": "detection of chemical stimulus involved in sensory perception of bitter taste",
  "gene_symbol": "TAS2R43",
  "gene_name": "Taste receptor type 2 member 43",
  "term_id": "GO:0001580"
}